{
  "gene_symbol": "TRIT1",
  "term_label": "tRNA dimethylallyltransferase activity",
  "term_id": "GO:0052381",
  "gene_name": "tRNA dimethylallyltransferase",
  "gene": "UniProtKB:Q9H3H1"
}